fruit morphogenesis [GO:0048530] (biological process) Definition: The process in which the anatomical structures of a fruit are generated and organized. A fruit is a reproductive body of a seed plant. Sources: GOC:sm Relationships: is a type of developmental process involved in reproduction [GO:0003006]; is a type of GO:0090698; is part of GO:0010154